aspartate carbamoyltransferase complex [GO:0009347] (cellular component) Note: Note that in eukaryotes, aspartate carbamoyltransferase is usually a single polypeptide, not a complex, and should therefore not be annotated to this component term. References: PMID:10447693 Definition: A multienzyme complex that catalyzes the formation N-carbamoyl-L-aspartate from carbamoyl phosphate and L-aspartate. It exhibits a variety of architectural organizations, but in all microorganisms the core catalytic component is a homotrimer of approximately 34 kDa polypeptides. Relationships: is a type of transferase complex [GO:1990234]